positive regulation of attachment of spindle microtubules to kinetochore [GO:0051987] (biological process) Subtypes: GO:1902425, GO:1904968 Also known as: up regulation of attachment of spindle microtubules to kinetochore, up-regulation of attachment of spindle microtubules to kinetochore, upregulation of attachment of spindle microtubules to kinetochore, activation of attachment of spindle microtubules to kinetochore, stimulation of attachment of spindle microtubules to kinetochore Relationships: is a type of GO:0051984; is_a regulation of attachment of spindle microtubules to kinetochore [GO:0051988]; positively regulates attachment of spindle microtubules to kinetochore [GO:0008608] Sources: GOC:ai Definition: Any process that activates or increases the frequency, rate or extent of the attachment of spindle microtubules to the kinetochore.